{
  "term_id": "GO:0016477",
  "gene_name": "Tyrosine-protein kinase receptor TYRO3",
  "gene": "UniProtKB:Q06418",
  "gene_symbol": "TYRO3",
  "term_label": "cell migration"
}